{
  "term_id": "GO:0005886",
  "term_label": "plasma membrane",
  "gene": "UniProtKB:Q8WXH2",
  "gene_name": "Junctophilin-3",
  "gene_symbol": "JPH3"
}